{
  "term_id": "UNKNOWN:0001",
  "term_label": "Unknown molecular function",
  "gene_symbol": "SPATA31A5",
  "gene": "UniProtKB:Q5VU36",
  "gene_name": "Spermatogenesis-associated protein 31A5"
}